{
  "term_label": "nucleus",
  "gene_name": "Zinc finger protein 181",
  "term_id": "GO:0005634",
  "gene": "UniProtKB:Q2M3W8",
  "gene_symbol": "ZNF181"
}